{
  "gene_name": "Homeobox protein Meis3",
  "term_label": "positive regulation of transcription by RNA polymerase II",
  "gene_symbol": "MEIS3",
  "gene": "UniProtKB:Q99687",
  "term_id": "GO:0045944"
}